{
  "term_id": "UNKNOWN:0001",
  "gene_name": "Centrosome-associated protein 350",
  "gene_symbol": "CEP350",
  "gene": "UniProtKB:Q5VT06",
  "term_label": "Unknown molecular function"
}